N-acetylglucosaminyldiphosphoundecaprenol glucosyltransferase activity [GO:0047245] (MF) Relationships: is a type of UDP-glucosyltransferase activity [GO:0035251] Also known as: UDP-D-glucose:N-acetylglucosaminyl pyrophosphorylundecaprenol glucosyltransferase activity, UDP-glucose:N-acetyl-D-glucosaminyldiphosphoundecaprenol 4-beta-D-glucosyltransferase activity, UDPglucose:N-acetyl-D-glucosaminyldiphosphoundecaprenol 4-beta-D-glucosyltransferase activity, uridine diphosphoglucose-acetylglucosaminylpyrophosphorylundecaprenol glucosyltransferase activity Sources: EC:2.4.1.188, MetaCyc:2.4.1.188-RXN Definition: Catalysis of the reaction: N-acetyl-D-glucosaminyldiphosphoundecaprenol + UDP-D-glucose = beta-D-glucosyl-1,4-N-acetyl-D-glucosaminyldiphosphoundecaprenol + UDP.